adenylate cyclase inhibitor activity [GO:0010855] (molecular function) Sources: GOC:dph, GOC:tb Relationships: is a type of cyclase inhibitor activity [GO:0010852]; is a type of adenylate cyclase regulator activity [GO:0010854]; negatively regulates adenylate cyclase activity [GO:0004016] Definition: Binds to and decreases the activity of adenylate cyclase.